{
  "gene_name": "Ankyrin-2",
  "gene": "UniProtKB:Q01484",
  "gene_symbol": "ANK2",
  "term_label": "plasma membrane",
  "term_id": "GO:0005886"
}